{
  "term_id": "GO:0015250",
  "term_label": "water channel activity",
  "gene": "UniProtKB:Q96PS8",
  "gene_name": "Aquaporin-10",
  "gene_symbol": "AQP10"
}